{
  "gene_symbol": "GJA10",
  "gene_name": "Gap junction alpha-10 protein",
  "term_id": "GO:0005922",
  "term_label": "connexin complex",
  "gene": "UniProtKB:Q969M2"
}